fertilization [GO:0009566] (biological process) Definition: The union of gametes of opposite sexes during the process of sexual reproduction to form a zygote. It involves the fusion of the gametic nuclei (karyogamy) and cytoplasm (plasmogamy). Sources: GOC:tb, ISBN:0198506732 Also known as: syngamy Relationships: is a type of reproductive process [GO:0022414]; is part of sexual reproduction [GO:0019953] Subtypes: single fertilization [GO:0007338], double fertilization forming a zygote and endosperm [GO:0009567], GO:0009677 Regulation: RO_0002212 by negative regulation of fertilization [GO:0060467]; regulated by regulation of fertilization [GO:0080154]; positively regulated by positive regulation of fertilization [GO:1905516]